{
  "term_id": "GO:0009952",
  "term_label": "anterior/posterior pattern specification",
  "gene_symbol": "HOXA5",
  "gene": "UniProtKB:P20719",
  "gene_name": "Homeobox protein Hox-A5"
}